{
  "term_id": "GO:0060090",
  "term_label": "molecular adaptor activity",
  "gene_symbol": "ARRDC3",
  "gene_name": "Arrestin domain-containing protein 3",
  "gene": "UniProtKB:Q96B67"
}